{
  "term_id": "GO:0097250",
  "gene_symbol": "HIGD1C",
  "term_label": "mitochondrial respirasome assembly",
  "gene_name": "HIG1 domain family member 1C",
  "gene": "UniProtKB:A8MV81"
}